positive regulation of gamma-aminobutyric acid secretion [GO:0014054] (biological process) Also known as: positive regulation of GABA secretion, up regulation of gamma-aminobutyric acid secretion, up-regulation of gamma-aminobutyric acid secretion, upregulation of gamma-aminobutyric acid secretion, activation of gamma-aminobutyric acid secretion, stimulation of gamma-aminobutyric acid secretion Sources: GOC:ef Definition: Any process that activates or increases the frequency, rate or extent of the regulated release of gamma-aminobutyric acid. Relationships: is a type of regulation of gamma-aminobutyric acid secretion [GO:0014052]; is a type of positive regulation of organic acid transport [GO:0032892]; is a type of GO:0051047; is_a GO:0051957; positively regulates gamma-aminobutyric acid secretion [GO:0014051]